{
  "term_id": "GO:0050808",
  "gene_symbol": "SNCG",
  "gene": "UniProtKB:O76070",
  "gene_name": "Gamma-synuclein",
  "term_label": "synapse organization"
}